{
  "gene_symbol": "ATOSB",
  "gene_name": "Atos homolog protein B",
  "gene": "UniProtKB:Q7L5A3",
  "term_label": "Unknown molecular function",
  "term_id": "UNKNOWN:0001"
}